{
  "gene_symbol": "VRK2",
  "term_label": "nucleus",
  "gene": "UniProtKB:Q86Y07",
  "term_id": "GO:0005634",
  "gene_name": "Serine_threonine-protein kinase VRK2"
}